{
  "gene": "UniProtKB:P08912",
  "gene_symbol": "CHRM5",
  "term_label": "plasma membrane",
  "term_id": "GO:0005886",
  "gene_name": "Muscarinic acetylcholine receptor M5"
}